type II terminal bouton [GO:0061175] (CC) Definition: Terminal inflated portion of the axon of a non-glutamatergic neuron, containing the specialized apparatus necessary to release neurotransmitters at a regulatory synapse. The axon terminus is considered to be the whole region of thickening and the terminal bouton is a specialized region of it. Sources: GOC:dph, GOC:mc Also known as: type II terminal button Relationships: is a type of terminal bouton [GO:0043195]